negative regulation of glycerol transport [GO:0090373] (BP) Sources: GOC:dph, GOC:jh, GOC:tb Relationships: is a type of negative regulation of transmembrane transport [GO:0034763]; is a type of regulation of glycerol transport [GO:0090371]; negatively regulates glycerol transmembrane transport [GO:0015793] Definition: Any process that decreases the rate, frequency, or extent of the directed movement of glycerol into, out of or within a cell, or between cells, by means of some agent such as a transporter or pore.